{
  "term_id": "UNKNOWN:0002",
  "gene_symbol": "NDUFB9",
  "term_label": "Unknown biological process",
  "gene": "UniProtKB:Q9Y6M9",
  "gene_name": "NADH dehydrogenase [ubiquinone] 1 beta subcomplex subunit 9"
}